{
  "gene_name": "Germ cell-specific gene 1-like protein 2",
  "term_label": "Unknown biological process",
  "gene": "UniProtKB:A8MUP6",
  "term_id": "UNKNOWN:0002",
  "gene_symbol": "GSG1L2"
}